{
  "term_label": "monoatomic cation homeostasis",
  "gene_name": "Protein unc-80 homolog",
  "term_id": "GO:0055080",
  "gene": "UniProtKB:Q8N2C7",
  "gene_symbol": "UNC80"
}